kanamycin kinase activity [GO:0008910] (molecular function) Sources: EC:2.7.1.95, RHEA:24256 Also known as: APH(3') activity, aminoglycoside 3'-phosphotransferase activity, ATP:kanamycin 3'-O-phosphotransferase activity, kanamycin kinase (phosphorylating), neomycin phosphotransferase activity, neomycin-kanamycin phosphotransferase activity Definition: Catalysis of the reaction: ATP + kanamycin = ADP + 2 H+ + kanamycin 3'-phosphate. Relationships: is a type of GO:0034071